{
  "term_label": "RNA binding",
  "gene_symbol": "NAF1",
  "gene": "UniProtKB:Q96HR8",
  "gene_name": "H_ACA ribonucleoprotein complex non-core subunit NAF1",
  "term_id": "GO:0003723"
}